{
  "term_label": "postsynaptic density",
  "gene_name": "SH2 domain-containing protein 5",
  "term_id": "GO:0014069",
  "gene": "UniProtKB:Q6ZV89",
  "gene_symbol": "SH2D5"
}